regulation of glucan biosynthetic process [GO:0010962] (biological process) Definition: Any process that modulates the rate, frequency, or extent of glucan biosynthesis. Glucan biosynthetic processes are the chemical reactions and pathways resulting in the formation of glucans, polysaccharides consisting only of glucose residues. Sources: GOC:dph, GOC:tb Relationships: is a type of GO:0032885; regulates glucan biosynthetic process [GO:0009250] Subtypes: regulation of glycogen biosynthetic process [GO:0005979], regulation of starch biosynthetic process [GO:0010581], regulation of alpha-glucan biosynthetic process [GO:0032949], regulation of beta-glucan biosynthetic process [GO:0032951]